serine family amino acid biosynthetic process [GO:0009070] (biological process) Subtypes: glycine biosynthetic process [GO:0006545], L-serine biosynthetic process [GO:0006564], homoserine biosynthetic process [GO:0009090], selenocysteine biosynthetic process [GO:0016260], cysteine biosynthetic process [GO:0019344], L-homocysteine biosynthetic process [GO:0071269] Also known as: serine family amino acid anabolism, serine family amino acid biosynthesis, serine family amino acid formation, serine family amino acid synthesis Relationships: is a type of alpha-amino acid biosynthetic process [GO:1901607] Sources: GOC:ai Definition: The chemical reactions and pathways resulting in the formation of amino acids of the serine family, comprising cysteine, glycine, homoserine, selenocysteine and serine.